{
  "term_id": "GO:0031721",
  "gene_name": "Hemoglobin subunit epsilon",
  "gene": "UniProtKB:P02100",
  "term_label": "hemoglobin alpha binding",
  "gene_symbol": "HBE1"
}